regulation of octopamine or tyramine signaling pathway [GO:2000125] (BP) Relationships: is a type of regulation of G protein-coupled receptor signaling pathway [GO:0008277]; regulates GO:0007211 Subtypes: negative regulation of octopamine or tyramine signaling pathway [GO:2000126], positive regulation of octopamine or tyramine signaling pathway [GO:2000127], regulation of octopamine signaling pathway [GO:2000128], regulation of tyramine signaling pathway [GO:2000131] Definition: Any process that modulates the frequency, rate or extent of octopamine or tyramine signaling pathway. Also known as: regulation of octopamine or tyramine signalling pathway, regulation of octopamine/tyramine signaling pathway Sources: GOC:mah